{
  "term_id": "GO:0004596",
  "gene_name": "N-alpha-acetyltransferase 20",
  "term_label": "protein-N-terminal amino-acid acetyltransferase activity",
  "gene": "UniProtKB:P61599",
  "gene_symbol": "NAA20"
}